{
  "term_id": "GO:0140912",
  "term_label": "membrane destabilizing activity",
  "gene_name": "Beta-defensin 123",
  "gene": "UniProtKB:Q8N688",
  "gene_symbol": "DEFB123"
}